{
  "gene": "UniProtKB:P14625",
  "gene_name": "Endoplasmin",
  "term_label": "endoplasmic reticulum",
  "gene_symbol": "HSP90B1",
  "term_id": "GO:0005783"
}